4-hydroxy-3-methylbut-2-enyl diphosphate reductase activity [GO:0051745] (molecular function) Also known as: 4-hydroxy-3-methylbut-2-en-1-yl diphosphate reductase activity, isopentenyl-diphosphate:NAD(P)+ oxidoreductase activity Definition: Catalyzes the conversion of (2E)-4-hydroxy-3-methylbut-2-enyl diphosphate + 2 H+ + 2 reduced [2Fe-2S]-[ferredoxin] to isopentenyl diphosphate (IPP) and dimethylallyl diphosphate (DMAPP) releasing H2O + 2 oxidized [2Fe-2S]-[ferredoxin]. Note that (E)-4-hydroxy-3-methylbut-2-en-1-yl diphosphate is an alternative name for 1-hydroxy-2-methyl-2-(E)-butenyl 4-diphosphate. Sources: EC:1.17.7.4, GOC:pg Relationships: is a type of oxidoreductase activity, acting on CH or CH2 groups, with an iron-sulfur protein as acceptor [GO:0052592]